{
  "gene_symbol": "USP3",
  "term_id": "UNKNOWN:0002",
  "gene_name": "Ubiquitin carboxyl-terminal hydrolase 3",
  "term_label": "Unknown biological process",
  "gene": "UniProtKB:Q9Y6I4"
}